{
  "term_id": "UNKNOWN:0002",
  "gene_symbol": "C2orf68",
  "gene": "UniProtKB:Q2NKX9",
  "term_label": "Unknown biological process",
  "gene_name": "UPF0561 protein C2orf68"
}